limb morphogenesis [GO:0035108] (biological process) Relationships: is a type of GO:0035107; is part of limb development [GO:0060173] Also known as: limb bud morphogenesis Sources: UBERON:0002101 Subtypes: embryonic limb morphogenesis [GO:0030326], post-embryonic limb morphogenesis [GO:0035127], GO:0035136, hindlimb morphogenesis [GO:0035137] Definition: The process in which the anatomical structures of a limb are generated and organized. A limb is a paired appendage of a tetrapod used for locomotion or grasping.